{
  "term_id": "UNKNOWN:0002",
  "term_label": "Unknown biological process",
  "gene_symbol": "MAB21L4",
  "gene": "UniProtKB:Q08AI8",
  "gene_name": "Protein mab-21-like 4"
}